cell migration in diencephalon [GO:0061381] (biological process) Sources: GOC:dph Definition: The orderly movement of a cell that will reside in the diencephalon. Relationships: is a type of forebrain cell migration [GO:0021885]; is part of diencephalon development [GO:0021536]